response to curcumin [GO:1904643] (biological process) Relationships: is a type of response to ether [GO:0045472]; is_a response to ketone [GO:1901654] Subtypes: cellular response to curcumin [GO:1904644] Definition: Any process that results in a change in state or activity of a cell or an organism (in terms of movement, secretion, enzyme production, gene expression, etc.) as a result of a curcumin stimulus. References: PMID:24755072 Sources: GOC:TermGenie, GO_REF:0000071